pyochelin biosynthetic process [GO:0042864] (BP) Relationships: is a type of siderophore biosynthetic process [GO:0019290]; is a type of sulfur compound biosynthetic process [GO:0044272]; is a type of phenol-containing compound biosynthetic process [GO:0046189]; is a type of carboxylic acid biosynthetic process [GO:0046394] References: PMID:6794030 Sources: GOC:jl Also known as: pyochelin anabolism, pyochelin biosynthesis, pyochelin formation, pyochelin synthesis, pyochelin biosynthetic process, peptide formation, pyochelin biosynthetic process, peptide modification Definition: The chemical reactions and pathways resulting in the formation of the siderochrome pyochelin (2-(2-o-hydroxyphenyl-2-thiazolin-4-yl)-3-methylthiazolidine-4-carboxylic acid).